dolichol phosphate mannose biosynthetic process [GO:0180047] (biological process) Definition: The chemical reactions and pathways resulting in the formation of dolichol phosphate mannose. Relationships: is a type of GO:0008654; is a type of glycolipid biosynthetic process [GO:0009247]; is a type of GO:0016114 Also known as: Dol-P-Man biosynthesis, dolichol phosphate mannose biosynthesis, dolichol-P-mannose biosynthesis References: PMID:18387370